{
  "term_id": "GO:0000151",
  "gene": "UniProtKB:Q9Y3C5",
  "term_label": "ubiquitin ligase complex",
  "gene_symbol": "RNF11",
  "gene_name": "RING finger protein 11"
}